{
  "term_id": "UNKNOWN:0002",
  "term_label": "Unknown biological process",
  "gene_symbol": "TMEM265",
  "gene": "UniProtKB:A0A087WTH1",
  "gene_name": "Transmembrane protein 265"
}